maintenance of meristem identity [GO:0010074] (biological process) Definition: The process in which an organism retains a population of meristem cells, preventing the commitment of all stem cell progeny to a differentiated cell fate. Sources: GOC:tb Also known as: maintenance of meristem cell identity, meristem cell maintenance Relationships: is a type of stem cell population maintenance [GO:0019827]; is part of GO:0010073 Subtypes: maintenance of floral meristem identity [GO:0010076], GO:0010077, maintenance of root meristem identity [GO:0010078], maintenance of vegetative meristem identity [GO:0010079], maintenance of shoot apical meristem identity [GO:0010492]